{
  "gene": "UniProtKB:Q0D2I5",
  "term_label": "Unknown molecular function",
  "term_id": "UNKNOWN:0001",
  "gene_symbol": "IFFO1",
  "gene_name": "Non-homologous end joining factor IFFO1"
}